response to cisplatin [GO:0072718] (biological process) Definition: Any process that results in a change in state or activity of a cell or an organism (in terms of movement, secretion, enzyme production, gene expression, etc.) as a result of a cisplatin stimulus. Relationships: is a type of response to chemical [GO:0042221] Subtypes: GO:0072719 Sources: GOC:mah